cordyol C metabolic process [GO:1900797] (biological process) Definition: The chemical reactions and pathways involving cordyol C. Sources: GOC:TermGenie, GOC:di Also known as: cordyol C metabolism Relationships: is a type of catechol-containing compound metabolic process [GO:0009712]; is a type of GO:0019748 Subtypes: cordyol C catabolic process [GO:1900798], cordyol C biosynthetic process [GO:1900799]